{
  "term_label": "lysosome localization",
  "gene": "UniProtKB:Q9NUM4",
  "term_id": "GO:0032418",
  "gene_name": "Transmembrane protein 106B",
  "gene_symbol": "TMEM106B"
}